{
  "term_label": "plasma membrane",
  "gene_name": "Olfactory receptor 10D3",
  "gene_symbol": "OR10D3",
  "term_id": "GO:0005886",
  "gene": "UniProtKB:Q8NH80"
}